negative regulation of IRE1-mediated unfolded protein response [GO:1903895] (biological process) References: PMID:22013210 Sources: GOC:PARL, GOC:TermGenie, GOC:bf, GO_REF:0000058 Relationships: is a type of GO:1900102; is a type of GO:1903894; negatively regulates IRE1-mediated unfolded protein response [GO:0036498] Also known as: down regulation of IRE1 branch of UPR, down regulation of IRE1-mediated unfolded protein response, down regulation of UPR signaling by IRE1 stress sensor, down regulation of endoplasmic reticulum unfolded protein response; IRE1 signaling, down-regulation of IRE1 branch of UPR, down-regulation of IRE1-mediated unfolded protein response, down-regulation of UPR signaling by IRE1 stress sensor, down-regulation of endoplasmic reticulum unfolded protein response; IRE1 signaling, downregulation of IRE1 branch of UPR, downregulation of IRE1-mediated unfolded protein response, downregulation of UPR signaling by IRE1 stress sensor, downregulation of endoplasmic reticulum unfolded protein response; IRE1 signaling, negative regulation of IRE1 branch of UPR, negative regulation of UPR signaling by IRE1 stress sensor, negative regulation of endoplasmic reticulum unfolded protein response; IRE1 signaling, down regulation of IRE1alpha unfolded protein response, down regulation of IRE1p unfolded protein response, down-regulation of IRE1alpha unfolded protein response, down-regulation of IRE1p unfolded protein response, downregulation of IRE1alpha unfolded protein response, downregulation of IRE1p unfolded protein response, inhibition of IRE1 branch of UPR, inhibition of IRE1-mediated unfolded protein response, inhibition of IRE1alpha unfolded protein response, inhibition of IRE1p unfolded protein response, inhibition of UPR signaling by IRE1 stress sensor, inhibition of endoplasmic reticulum unfolded protein response; IRE1 signaling, negative regulation of IRE1alpha unfolded protein response, negative regulation of IRE1p unfolded protein response, down regulation of IRE1 signaling in response to endoplasmic reticulum stress, down regulation of inositol-requiring transmembrane kinase/endonuclease signal transduction, down-regulation of IRE1 signaling in response to endoplasmic reticulum stress, down-regulation of inositol-requiring transmembrane kinase/endonuclease signal transduction, downregulation of IRE1 signaling in response to endoplasmic reticulum stress, downregulation of inositol-requiring transmembrane kinase/endonuclease signal transduction, inhibition of IRE1 signaling in response to endoplasmic reticulum stress, inhibition of inositol-requiring transmembrane kinase/endonuclease signal transduction, negative regulation of ERN1-mediated unfolded protein response, negative regulation of IRE1 signaling in response to endoplasmic reticulum stress, negative regulation of inositol-requiring transmembrane kinase/endonuclease signal transduction Definition: Any process that stops, prevents or reduces the frequency, rate or extent of the IRE1-mediated unfolded protein response.